{
  "gene_name": "Brain-derived neurotrophic factor",
  "term_label": "modulation of chemical synaptic transmission",
  "gene_symbol": "BDNF",
  "gene": "UniProtKB:P23560",
  "term_id": "GO:0050804"
}